{
  "gene_symbol": "MGST3",
  "term_label": "Unknown biological process",
  "gene": "UniProtKB:O14880",
  "term_id": "UNKNOWN:0002",
  "gene_name": "Glutathione S-transferase 3, mitochondrial"
}